{
  "gene_symbol": "SLC35F3",
  "term_label": "Unknown cellular component",
  "gene": "UniProtKB:Q8IY50",
  "gene_name": "Solute carrier family 35 member F3",
  "term_id": "UNKNOWN:0003"
}